{
  "gene_symbol": "EXD3",
  "gene": "UniProtKB:Q8N9H8",
  "term_id": "UNKNOWN:0002",
  "gene_name": "Exonuclease mut-7 homolog",
  "term_label": "Unknown biological process"
}